{
  "gene_symbol": "PPP1R10",
  "term_label": "enzyme-substrate adaptor activity",
  "gene": "UniProtKB:Q96QC0",
  "term_id": "GO:0140767",
  "gene_name": "Serine_threonine-protein phosphatase 1 regulatory subunit 10"
}